{
  "gene": "UniProtKB:Q07955",
  "gene_symbol": "SRSF1",
  "term_label": "mRNA binding",
  "gene_name": "Serine_arginine-rich splicing factor 1",
  "term_id": "GO:0003729"
}